basolateral recycling endosome [GO:0090654] (cellular component) Definition: Tubulo-vesicular structure located in the basolateral cytoplasm that participates in basolateral cargo recycling in polarized epithelial cells. References: PMID:11389442, PMID:16394106, PMID:17494872, PMID:21170358, PMID:9405315 Relationships: is a type of GO:0055037; is part of basolateral cytoplasm [GO:0090652]